{
  "gene": "UniProtKB:Q9P219",
  "term_label": "cytoplasm",
  "gene_symbol": "CCDC88C",
  "term_id": "GO:0005737",
  "gene_name": "Protein Daple"
}